negative regulation of glial cell-derived neurotrophic factor production [GO:1900167] (biological process) Also known as: negative regulation of GDNF secretion, inhibition of GDNF secretion, inhibition of glial cell line-derived neurotrophic factor secretion, negative regulation of glial cell-derived neurotrophic factor secretion, negative regulation of glial cell line-derived neurotrophic factor secretion Relationships: is_a negative regulation of cytokine production [GO:0001818]; is a type of regulation of glial cell-derived neurotrophic factor production [GO:1900166]; negatively regulates GO:0044467 Sources: GOC:TermGenie, GOC:yaf Definition: Any process that stops, prevents or reduces the frequency, rate or extent of glial cell-derived neurotrophic factor production.